{
  "gene_name": "Guanine nucleotide-binding protein G(t) subunit alpha-1",
  "term_label": "detection of light stimulus involved in visual perception",
  "term_id": "GO:0050908",
  "gene": "UniProtKB:P11488",
  "gene_symbol": "GNAT1"
}